{
  "gene_name": "UBX domain-containing protein 7",
  "term_label": "nucleus",
  "gene": "UniProtKB:O94888",
  "term_id": "GO:0005634",
  "gene_symbol": "UBXN7"
}